{
  "gene": "UniProtKB:Q9UHA3",
  "gene_symbol": "RSL24D1",
  "term_label": "Unknown molecular function",
  "term_id": "UNKNOWN:0001",
  "gene_name": "Probable ribosome biogenesis protein RLP24"
}